{
  "term_label": "phospholipid binding",
  "gene_name": "MYCBP-associated protein",
  "term_id": "GO:0005543",
  "gene": "UniProtKB:Q8TBZ2",
  "gene_symbol": "MYCBPAP"
}